{
  "gene_name": "Cullin-4B",
  "gene": "UniProtKB:Q13620",
  "term_label": "Cul4B-RING E3 ubiquitin ligase complex",
  "term_id": "GO:0031465",
  "gene_symbol": "CUL4B"
}